{
  "gene_name": "CCR4-NOT transcription complex subunit 1",
  "term_label": "P-body",
  "gene_symbol": "CNOT1",
  "term_id": "GO:0000932",
  "gene": "UniProtKB:A5YKK6"
}